negative regulation of cell adhesion involved in substrate-bound cell migration [GO:0006933] (biological process) Definition: The disassembly of adhesions at the front and rear of a migrating cell. At the leading edge, adhesion disassembly accompanies the formation of new protrusions; at the cell rear, it promotes tail retraction. References: PMID:11944043, PMID:14657486 Sources: GOC:dph, GOC:tb, ISBN:0815316194 Also known as: substrate-bound cell migration, cell release from substrate Relationships: is a type of GO:0007162; is part of substrate-dependent cell migration [GO:0006929]